{
  "term_id": "GO:0031463",
  "term_label": "Cul3-RING ubiquitin ligase complex",
  "gene_symbol": "KLHL18",
  "gene_name": "Kelch-like protein 18",
  "gene": "UniProtKB:O94889"
}